cellular detoxification of sulfide [GO:0140974] (biological process) Definition: Any process carried out at the cellular level that reduces or removes the toxicity of a sulfide. These may include chemical modification or transport of sulfide away from sensitive areas and to compartments or complexes whose purpose is sequestration of the toxic substance. References: PMID:20077566, PMID:25747485 Relationships: is a type of cellular detoxification [GO:1990748]